spinal cord oligodendrocyte cell differentiation [GO:0021529] (biological process) Relationships: is a type of GO:0021515; is a type of GO:0048709 Definition: The process in which neuroepithelial cells in the neural tube acquire specialized structural and/or functional features of oligodendrocytes. Oligodendrocytes are non-neuronal cells. The primary function of oligodendrocytes is the myelination of nerve axons in the central nervous system. Differentiation includes the processes involved in commitment of a cell to a specific fate. Sources: GOC:cls, GOC:dgh, GOC:dph, GOC:jid, GO_REF:0000021